{
  "gene_symbol": "MTRR",
  "gene": "UniProtKB:Q9UBK8",
  "term_id": "GO:0010181",
  "term_label": "FMN binding",
  "gene_name": "Methionine synthase reductase"
}